{
  "gene": "UniProtKB:Q9H2A9",
  "term_id": "GO:0008146",
  "gene_symbol": "CHST8",
  "gene_name": "Carbohydrate sulfotransferase 8",
  "term_label": "sulfotransferase activity"
}